{
  "term_id": "GO:0045944",
  "gene_symbol": "GATA3",
  "gene_name": "Trans-acting T-cell-specific transcription factor GATA-3",
  "term_label": "positive regulation of transcription by RNA polymerase II",
  "gene": "UniProtKB:P23771"
}